{
  "gene_name": "Zinc finger protein ZFPM1",
  "term_id": "GO:0030219",
  "gene_symbol": "ZFPM1",
  "term_label": "megakaryocyte differentiation",
  "gene": "UniProtKB:Q8IX07"
}